{
  "term_id": "GO:0000064",
  "term_label": "L-ornithine transmembrane transporter activity",
  "gene": "UniProtKB:P30825",
  "gene_name": "High affinity cationic amino acid transporter 1",
  "gene_symbol": "SLC7A1"
}